{
  "term_id": "GO:0007608",
  "term_label": "sensory perception of smell",
  "gene_name": "Olfactory receptor 5D13",
  "gene": "UniProtKB:Q8NGL4",
  "gene_symbol": "OR5D13"
}